bundle of His cell to Purkinje myocyte communication [GO:0086069] (biological process) Also known as: bundle of His cardiac muscle cell to Purkinje myocyte communication, ventricular conduction system cell to cell communication, atrioventricular junction myocyte to bundle branch myocyte, bundle branch myocyte to Purkinje myocyte communication, bundle of His myocyte to atrioventricular junction myocyte Subtypes: bundle of His cell to Purkinje myocyte signaling [GO:0086028], bundle of His cell to Purkinje myocyte communication by electrical coupling [GO:0086054] Relationships: is a type of cell communication involved in cardiac conduction [GO:0086065] Sources: GOC:BHF, GOC:mtg_cardiac_conduct_nov11 Definition: The process that mediates interactions between a bundle of His cell and its surroundings that contributes to the process of the bundle of His cell communicating with a Purkinje myocyte in cardiac conduction. Encompasses interactions such as signaling or attachment between one cell and another cell, between a cell and an extracellular matrix, or between a cell and any other aspect of its environment.